{
  "term_id": "UNKNOWN:0002",
  "gene_symbol": "PNMA1",
  "gene": "UniProtKB:Q8ND90",
  "gene_name": "Paraneoplastic antigen Ma1",
  "term_label": "Unknown biological process"
}